lymphocyte costimulation [GO:0031294] (biological process) Relationships: is a type of GO:0002376; is a type of GO:0051251 Sources: ISBN:0781735149 Definition: The process of providing, via surface-bound receptor-ligand pairs, a second, antigen-independent, signal in addition to that provided by the B- or T cell receptor to augment B- or T cell activation. Subtypes: T cell costimulation [GO:0031295], B cell costimulation [GO:0031296] Also known as: lymphocyte co-stimulation